L-cysteine catabolic process via cystine, using cysteine transaminase [GO:0019456] (BP) Also known as: L-cysteine breakdown via cystine, using cysteine transaminase, L-cysteine degradation via cystine, using cysteine transaminase Relationships: is a type of L-cysteine catabolic process via cystine [GO:0019453]; has part L-cysteine transaminase activity [GO:0047801] Definition: The chemical reactions and pathways resulting in the breakdown, via the compound cystine, of L-cysteine, catalyzed by the enzyme cysteine transaminase. Sources: GOC:jl